{
  "term_id": "GO:0000398",
  "gene_name": "U6 snRNA-associated Sm-like protein LSm6",
  "gene_symbol": "LSM6",
  "term_label": "mRNA splicing, via spliceosome",
  "gene": "UniProtKB:P62312"
}